{
  "gene": "UniProtKB:Q6ZVH6",
  "gene_name": "Putative uncharacterized protein FLJ42569",
  "term_id": "UNKNOWN:0003",
  "term_label": "Unknown cellular component",
  "gene_symbol": "Q6ZVH6"
}